{
  "gene": "UniProtKB:P50749",
  "term_label": "positive regulation of JNK cascade",
  "gene_symbol": "RASSF2",
  "gene_name": "Ras association domain-containing protein 2",
  "term_id": "GO:0046330"
}